histone H4K20 trimethyltransferase activity [GO:0140943] (molecular function) Definition: Catalysis of the reaction: L-lysyl(20)-[histone H4] + 3 S-adenosyl-L-methionine = 3 H+ + N(6),N(6),N(6)-trimethyl-L-lysyl(20)-[histone H4] + 3 S-adenosyl-L-homocysteine. This reaction is the addition of three methyl groups to the lysine residue at position 20 of the histone H4 protein, producing histone H4K20me3. Relationships: is a type of histone H4K20 methyltransferase activity [GO:0042799] Note: Note that the residue position corresponds to the canonical human H4 histone (UniProtKB:P02309); this residue is conserved across all eukaryotes. Note that the initiation methionine is cleaved, so the first residue is S1. Also known as: histone H4K20 trimethylase activity, histone H4K20 trimethylation, histone lysine N-trimethyltransferase activity (H4-K20 specific) Sources: RHEA:64456